{
  "term_id": "UNKNOWN:0001",
  "term_label": "Unknown molecular function",
  "gene_symbol": "CDKL5",
  "gene": "UniProtKB:O76039",
  "gene_name": "Cyclin-dependent kinase-like 5"
}